{
  "gene_symbol": "WRAP73",
  "term_label": "microtubule anchoring at mitotic spindle pole body",
  "gene": "UniProtKB:Q9P2S5",
  "gene_name": "WD repeat-containing protein WRAP73",
  "term_id": "GO:1990810"
}